{
  "gene_name": "MOB kinase activator 3B",
  "gene": "UniProtKB:Q86TA1",
  "term_label": "signal transduction",
  "gene_symbol": "MOB3B",
  "term_id": "GO:0007165"
}